{
  "term_id": "GO:0045661",
  "gene_symbol": "FLOT2",
  "gene": "UniProtKB:Q14254",
  "term_label": "regulation of myoblast differentiation",
  "gene_name": "Flotillin-2"
}